L-glutamate catabolic process [GO:0006538] (biological process) Sources: GOC:go_curators Relationships: is a type of glutamate metabolic process [GO:0006536]; is a type of dicarboxylic acid catabolic process [GO:0043649]; is a type of GO:0170035; is a type of proteinogenic amino acid catabolic process [GO:0170040] Also known as: glutamate breakdown, glutamate catabolism, glutamate degradation, glutamic acid catabolic process, glutamic acid catabolism, glutamate deamidation Subtypes: gamma-aminobutyrate shunt [GO:0006540], L-glutamate catabolic process to aspartate [GO:0019550], L-glutamate catabolic process via L-citramalate [GO:0019553], GO:0019555, anaerobic L-glutamate catabolic process [GO:0019670], L-glutamate catabolic process to butyrate [GO:0033508], L-glutamate catabolic process to propionate [GO:0033509], glutamate catabolic process to 4-hydroxybutyrate [GO:0036241] Definition: The chemical reactions and pathways resulting in the breakdown of L-glutamate, the anion of 2-aminopentanedioic acid.